{
  "term_label": "embryonic cranial skeleton morphogenesis",
  "gene": "UniProtKB:P16234",
  "term_id": "GO:0048701",
  "gene_symbol": "PDGFRA",
  "gene_name": "Platelet-derived growth factor receptor alpha"
}